{
  "term_label": "mRNA 3'-UTR binding",
  "gene": "UniProtKB:P29558",
  "term_id": "GO:0003730",
  "gene_symbol": "RBMS1",
  "gene_name": "RNA-binding motif, single-stranded-interacting protein 1"
}